{
  "gene_name": "Olfactory receptor 12D2",
  "gene": "UniProtKB:P58182",
  "term_label": "odorant binding",
  "term_id": "GO:0005549",
  "gene_symbol": "OR12D2"
}